{
  "term_id": "UNKNOWN:0001",
  "gene_name": "POTE ankyrin domain family member C",
  "term_label": "Unknown molecular function",
  "gene_symbol": "POTEC",
  "gene": "UniProtKB:B2RU33"
}